{
  "gene_symbol": "CD86",
  "gene_name": "T-lymphocyte activation antigen CD86",
  "gene": "UniProtKB:P42081",
  "term_label": "T cell costimulation",
  "term_id": "GO:0031295"
}